regulation of olefin biosynthetic process [GO:1900911] (biological process) Definition: Any process that modulates the frequency, rate or extent of olefin biosynthetic process. Sources: GOC:TermGenie, GOC:mengo_curators Also known as: regulation of olefin anabolism, regulation of olefin biosynthesis, regulation of olefin formation, regulation of olefin synthesis Relationships: is a type of regulation of biosynthetic process [GO:0009889]; RO_0002211 olefin biosynthetic process [GO:1900674] Subtypes: GO:0010364, negative regulation of olefin biosynthetic process [GO:1900912], positive regulation of olefin biosynthetic process [GO:1900913], GO:1900914, GO:1900935, regulation of (Z)-nonadeca-1,14-diene biosynthetic process [GO:1900941], regulation of isoprene biosynthetic process [GO:1900947], regulation of 18-methylnonadec-1-ene biosynthetic process [GO:1900950], regulation of 17-methylnonadec-1-ene biosynthetic process [GO:1900956]